{
  "gene_name": "Adenylate kinase 2, mitochondrial",
  "gene_symbol": "AK2",
  "term_id": "GO:0005739",
  "gene": "UniProtKB:P54819",
  "term_label": "mitochondrion"
}